{
  "term_label": "ruffle assembly",
  "gene_symbol": "AIF1L",
  "gene_name": "Allograft inflammatory factor 1-like",
  "gene": "UniProtKB:Q9BQI0",
  "term_id": "GO:0097178"
}